cytotoxic T cell pyroptotic cell death [GO:1902483] (biological process) Definition: A pyroptotic cell death process that occurs in a cytotoxic T cell. References: PMID:32299851 Also known as: cytotoxic T cell pyroptotic process, cytotoxic T cell apoptosis, cytotoxic T cell apoptotic process, cytotoxic T lymphocyte apoptotic process, cytotoxic T-cell apoptosis, cytotoxic T-cell programmed cell death Relationships: is a type of pyroptotic cell death [GO:0141201]